{
  "term_id": "GO:0001817",
  "gene_name": "Zinc finger protein 134",
  "term_label": "regulation of cytokine production",
  "gene_symbol": "ZNF134",
  "gene": "UniProtKB:P52741"
}